{
  "gene_name": "Large ribosomal subunit protein mL66",
  "term_label": "small ribosomal subunit rRNA binding",
  "term_id": "GO:0070181",
  "gene": "UniProtKB:Q9NVS2",
  "gene_symbol": "MRPS18A"
}